{
  "gene": "UniProtKB:O75508",
  "term_label": "Unknown molecular function",
  "term_id": "UNKNOWN:0001",
  "gene_name": "Claudin-11",
  "gene_symbol": "CLDN11"
}